orsellinate-depside hydrolase activity [GO:0050160] (molecular function) Relationships: is a type of carboxylic ester hydrolase activity [GO:0052689] Also known as: lecanorate hydrolase activity Definition: Catalysis of the reaction: H2O + orsellinate depside = 2 o-orsellinate + H+. Sources: EC:3.1.1.40, RHEA:19549